glutamate-methylamine ligase activity [GO:0047943] (molecular function) Definition: Catalysis of the reaction: L-glutamate + ATP + methylammonium = N(5)-methyl-L-glutamine + ADP + 2 H+ + phosphate. Also known as: L-glutamate:methylamine ligase (ADP-forming), gamma-glutamylmethylamide synthetase activity Relationships: is a type of GO:0016879 Sources: EC:6.3.4.12, RHEA:17117